{
  "term_id": "GO:0007411",
  "gene_symbol": "PLEKHG4",
  "gene": "UniProtKB:Q58EX7",
  "term_label": "axon guidance",
  "gene_name": "Puratrophin-1"
}